{
  "gene_name": "Aggrecan core protein",
  "term_id": "GO:0001501",
  "gene": "UniProtKB:P16112",
  "term_label": "skeletal system development",
  "gene_symbol": "ACAN"
}